{
  "term_label": "positive regulation of cell population proliferation",
  "gene_name": "Lithostathine-1-beta",
  "term_id": "GO:0008284",
  "gene": "UniProtKB:P48304",
  "gene_symbol": "REG1B"
}